{
  "gene": "UniProtKB:O95460",
  "gene_symbol": "MATN4",
  "term_id": "UNKNOWN:0002",
  "term_label": "Unknown biological process",
  "gene_name": "Matrilin-4"
}